{
  "gene_name": "Testis-expressed protein 264",
  "gene": "UniProtKB:Q9Y6I9",
  "term_label": "nucleus",
  "term_id": "GO:0005634",
  "gene_symbol": "TEX264"
}